{
  "gene_symbol": "MLIP",
  "term_id": "UNKNOWN:0003",
  "gene": "UniProtKB:Q5VWP3",
  "gene_name": "Muscular LMNA-interacting protein",
  "term_label": "Unknown cellular component"
}